{
  "gene_symbol": "IGSF9",
  "gene": "UniProtKB:Q9P2J2",
  "term_id": "GO:0070593",
  "gene_name": "Protein turtle homolog A",
  "term_label": "dendrite self-avoidance"
}